{
  "term_label": "negative regulation of microtubule polymerization",
  "gene": "UniProtKB:Q15735",
  "gene_name": "Phosphatidylinositol 4,5-bisphosphate 5-phosphatase A",
  "gene_symbol": "INPP5J",
  "term_id": "GO:0031115"
}